complement component C3d binding [GO:0001854] (molecular function) Definition: Binding to a C3d product of the complement cascade. Sources: GOC:add, ISBN:0781735149 Relationships: is a type of complement binding [GO:0001848]